{
  "term_label": "Unknown cellular component",
  "gene_symbol": "ZFAND5",
  "gene": "UniProtKB:O76080",
  "term_id": "UNKNOWN:0003",
  "gene_name": "AN1-type zinc finger protein 5"
}